short-term synaptic potentiation [GO:1990926] (biological process) References: PMID:11826273, PMID:26738595 Sources: GOC:dos, GOC:sp, ISBN:9780071120005 Note: The mechanism of short term potentiation is thought to be either increased influx of calcium into the presynapse (Zucker and Regeh, 2002 PMID:11826273) increased sensitivity to calcium (Jackman et al., 2016 PMID:26738595) or both. Relationships: is a type of regulation of synaptic plasticity [GO:0048167] Also known as: synaptic facilitation Regulation: regulated by regulation of short-term synaptic potentiation [GO:1905512]; negatively regulated by negative regulation of short-term synaptic potentiation [GO:1905513]; positively regulated by positive regulation of short-term synaptic potentiation [GO:1905514] Definition: The process by which synaptic transmission, induced by the arrival of a spike (action potential) at a synapse, acts to increase the amount of neurotransmitter released in response to the arrival of subsequent spikes. This effect is seen when a train of closely space spikes arrives at a synapse with a low initial release probability. It occurs in a timeframe of tens to hundreds of milliseconds.